{
  "gene_symbol": "RUVBL2",
  "term_label": "regulation of transcription by RNA polymerase II",
  "gene": "UniProtKB:Q9Y230",
  "term_id": "GO:0006357",
  "gene_name": "RuvB-like 2"
}